extracellular matrix-granule cell signaling involved in regulation of granule cell precursor proliferation [GO:0021939] (biological process) Relationships: is a type of extracellular matrix-cell signaling [GO:0035426]; is part of negative regulation of cerebellar granule cell precursor proliferation [GO:0021941] References: PMID:15157725 Sources: GOC:cls, GOC:dgh, GOC:dph, GOC:jid, GO_REF:0000021 Definition: The process that mediates the transfer of information from the extracellular matrix to granule cell precursors resulting in a decrease in rate of granule cell precursor cell proliferation. Also known as: extracellular matrix-granule cell signalling involved in regulation of granule cell precursor proliferation